{
  "gene_symbol": "ABCC10",
  "term_id": "GO:0055085",
  "gene_name": "ATP-binding cassette sub-family C member 10",
  "gene": "UniProtKB:Q5T3U5",
  "term_label": "transmembrane transport"
}